{
  "term_id": "UNKNOWN:0001",
  "term_label": "Unknown molecular function",
  "gene": "UniProtKB:Q12816",
  "gene_symbol": "TRO",
  "gene_name": "Trophinin"
}